{
  "term_id": "GO:0038023",
  "gene": "UniProtKB:Q6NUI6",
  "gene_name": "Chondroadherin-like protein",
  "gene_symbol": "CHADL",
  "term_label": "signaling receptor activity"
}